{
  "gene_name": "Ubiquinol-cytochrome-c reductase complex assembly factor 1",
  "gene": "UniProtKB:Q9NVA1",
  "term_id": "UNKNOWN:0001",
  "term_label": "Unknown molecular function",
  "gene_symbol": "UQCC1"
}